{
  "term_label": "cytosol",
  "term_id": "GO:0005829",
  "gene": "UniProtKB:A0A1W2PR95",
  "gene_symbol": "IGBP1C",
  "gene_name": "Immunoglobulin-binding protein 1 family member C"
}